{
  "term_label": "Unknown molecular function",
  "gene_name": "G-protein coupled receptor-associated sorting protein 1",
  "gene": "UniProtKB:Q5JY77",
  "term_id": "UNKNOWN:0001",
  "gene_symbol": "GPRASP1"
}